phyllome development [GO:0048827] (biological process) Subtypes: bract development [GO:0010432], leaf development [GO:0048366], carpel development [GO:0048440], petal development [GO:0048441], sepal development [GO:0048442], stamen development [GO:0048443] Sources: GOC:devbiol, GOC:tb, PO:0006001 Relationships: is a type of plant organ development [GO:0099402]; is part of shoot system development [GO:0048367] Definition: The process whose specific outcome is the progression of a phyllome over time, from its formation to the mature structure. A phyllome is a collective term for all the different types of leaves appearing on plants.